{
  "gene_symbol": "TUBB3",
  "gene": "UniProtKB:Q13509",
  "gene_name": "Tubulin beta-3 chain",
  "term_label": "GTP binding",
  "term_id": "GO:0005525"
}